{
  "term_id": "UNKNOWN:0001",
  "gene_symbol": "XKRX",
  "gene": "UniProtKB:Q6PP77",
  "gene_name": "XK-related protein 2",
  "term_label": "Unknown molecular function"
}